{
  "term_id": "GO:0005886",
  "term_label": "plasma membrane",
  "gene": "UniProtKB:Q8NGJ3",
  "gene_name": "Olfactory receptor 52E1",
  "gene_symbol": "OR52E1"
}